embryonic cleavage [GO:0040016] (biological process) Relationships: is a type of cell division [GO:0051301]; is part of GO:0009790 Sources: GOC:clt, ISBN:0070524300 Definition: The first few specialized divisions of an activated animal egg.